{
  "gene_symbol": "KAZALD1",
  "term_id": "GO:0005615",
  "term_label": "extracellular space",
  "gene_name": "Kazal-type serine protease inhibitor domain-containing protein 1",
  "gene": "UniProtKB:Q96I82"
}